cellular response to cortisol stimulus [GO:0071387] (biological process) Relationships: is a type of response to cortisol [GO:0051414]; is a type of cellular response to glucocorticoid stimulus [GO:0071385]; is a type of GO:0097306; is a type of cellular response to ketone [GO:1901655] Definition: Any process that results in a change in state or activity of a cell (in terms of movement, secretion, enzyme production, gene expression, etc.) as a result of a cortisol stimulus. Cortisol is the major natural glucocorticoid synthesized in the zona fasciculata of the adrenal cortex; it affects the metabolism of glucose, protein, and fats and has appreciable mineralocorticoid activity. It also regulates the immune system and affects many other functions. Also known as: cellular response to hydrocortisone stimulus Sources: GOC:mah